{
  "gene": "UniProtKB:Q8NFJ8",
  "term_label": "positive regulation of transcription by RNA polymerase II",
  "term_id": "GO:0045944",
  "gene_symbol": "BHLHE22",
  "gene_name": "Class E basic helix-loop-helix protein 22"
}